{
  "term_label": "Unknown biological process",
  "gene": "UniProtKB:Q9Y3A2",
  "term_id": "UNKNOWN:0002",
  "gene_name": "Probable U3 small nucleolar RNA-associated protein 11",
  "gene_symbol": "UTP11"
}